matrix side of mitochondrial inner membrane [GO:0099617] (cellular component) Relationships: is a type of lumenal side of membrane [GO:0098576]; is part of mitochondrial inner membrane [GO:0005743] Definition: The side (leaflet) of the mitochondrial inner membrane that faces the matrix. Sources: GOC:dos